{
  "term_label": "RNA polymerase II cis-regulatory region sequence-specific DNA binding",
  "gene_symbol": "HELT",
  "term_id": "GO:0000978",
  "gene_name": "Hairy and enhancer of split-related protein HELT",
  "gene": "UniProtKB:A6NFD8"
}